{
  "term_label": "photoreceptor outer segment",
  "gene": "UniProtKB:P08100",
  "gene_name": "Rhodopsin",
  "gene_symbol": "RHO",
  "term_id": "GO:0001750"
}